{
  "gene_symbol": "FGF16",
  "term_id": "GO:0008543",
  "gene_name": "Fibroblast growth factor 16",
  "term_label": "fibroblast growth factor receptor signaling pathway",
  "gene": "UniProtKB:O43320"
}